L-pipecolic acid biosynthetic process [GO:0062034] (biological process) Definition: The chemical reactions and pathways resulting in the formation of L-pipecolic acid, a metabolite of lysine. References: PMID:27758894, PMID:28330936 Relationships: is a type of monocarboxylic acid biosynthetic process [GO:0072330] Also known as: L-pipecolate biosynthetic process